regulation of L-proline metabolic process [GO:2000214] (biological process) Sources: GOC:sl Subtypes: GO:1902005, regulation of L-proline catabolic process to L-glutamate [GO:2001156] Definition: Any process that modulates the frequency, rate or extent of L-proline metabolic process. Also known as: regulation of proline metabolic process, regulation of proline metabolism Relationships: is a type of regulation of amino acid metabolic process [GO:0006521]; is_a regulation of small molecule metabolic process [GO:0062012]; regulates GO:0006560